{
  "gene": "UniProtKB:Q8NGL7",
  "term_id": "GO:0005886",
  "term_label": "plasma membrane",
  "gene_name": "Olfactory receptor 4P4",
  "gene_symbol": "OR4P4"
}